{
  "gene_name": "Nesprin-3",
  "term_label": "meiotic nuclear membrane microtubule tethering complex",
  "term_id": "GO:0034993",
  "gene": "UniProtKB:Q6ZMZ3",
  "gene_symbol": "SYNE3"
}